regulation of asexual reproduction [GO:1903664] (biological process) Definition: Any process that modulates the frequency, rate or extent of asexual reproduction. Subtypes: regulation of cell budding [GO:0007116], regulation of asexual sporulation [GO:0034305], GO:1903665, positive regulation of asexual reproduction [GO:1903666] Relationships: is a type of regulation of reproductive process [GO:2000241]; regulates asexual reproduction [GO:0019954] References: PMID:24390142 Sources: GOC:TermGenie, GO_REF:0000058